{
  "term_label": "regulation of alternative mRNA splicing, via spliceosome",
  "term_id": "GO:0000381",
  "gene_symbol": "CELF4",
  "gene": "UniProtKB:Q9BZC1",
  "gene_name": "CUGBP Elav-like family member 4"
}